regulation of mitochondrial translational initiation [GO:0070132] (biological process) Definition: Any process that modulates the frequency, rate or extent of the process preceding formation of the peptide bond between the first two amino acids of a protein in a mitochondrion. Also known as: regulation of mitochondrial translation initiation Subtypes: negative regulation of mitochondrial translational initiation [GO:0070133], positive regulation of mitochondrial translational initiation [GO:0070134] Relationships: is a type of regulation of translational initiation [GO:0006446]; is a type of GO:0070129; regulates mitochondrial translational initiation [GO:0070124] Sources: GOC:mah